cytoplasmic U snRNP body assembly [GO:1990194] (biological process) Also known as: U body assembly Relationships: is a type of protein-RNA complex assembly [GO:0022618]; is a type of membraneless organelle assembly [GO:0140694] Definition: The aggregation, arrangement and bonding together of proteins and RNA molecules to form a cytoplasmic U snRNP body. References: PMID:19464282